regulation of intracellular sterol transport [GO:0032380] (biological process) Subtypes: negative regulation of intracellular sterol transport [GO:0032381], GO:0032382, GO:0032383 Sources: GOC:mah Definition: Any process that modulates the frequency, rate or extent of the directed movement of sterols within cells. Relationships: is a type of regulation of sterol transport [GO:0032371]; is a type of regulation of intracellular lipid transport [GO:0032377]; regulates intracellular sterol transport [GO:0032366]